{
  "gene_symbol": "STOML2",
  "term_id": "GO:0005739",
  "gene_name": "Stomatin-like protein 2, mitochondrial",
  "term_label": "mitochondrion",
  "gene": "UniProtKB:Q9UJZ1"
}